positive regulation of flagellated sperm motility [GO:1902093] (biological process) Subtypes: GO:0060474 Relationships: is a type of positive regulation of cilium movement [GO:0003353]; is a type of regulation of flagellated sperm motility [GO:1901317]; is a type of positive regulation of cilium-dependent cell motility [GO:2000155]; is a type of positive regulation of reproductive process [GO:2000243]; positively regulates flagellated sperm motility [GO:0030317] Also known as: activation of sperm movement, positive regulation of sperm motility, positive regulation of sperm movement, up regulation of sperm motility, up regulation of sperm movement, up-regulation of sperm motility, up-regulation of sperm movement, upregulation of sperm motility, upregulation of sperm movement, activation of sperm motility References: PMID:7513657 Sources: GOC:TermGenie, GOC:cilia, GOC:jh2, GOC:krc Definition: Any process that activates or increases the frequency, rate or extent of flagellated sperm motility.